indolalkylamine biosynthetic process [GO:0046219] (biological process) Sources: GOC:curators Definition: The chemical reactions and pathways resulting in the formation of indolalkylamines, indole or indole derivatives containing a primary, secondary, or tertiary amine group. Relationships: is a type of biogenic amine biosynthetic process [GO:0042401]; is a type of indole-containing compound biosynthetic process [GO:0042435] Also known as: indolalkylamine anabolism, indolalkylamine biosynthesis, indolalkylamine formation, indolalkylamine synthesis Subtypes: L-tryptophan biosynthetic process [GO:0000162]